phytochromobilin biosynthetic process [GO:0010024] (biological process) References: PMID:11402195 Also known as: phytochromobilin anabolism, phytochromobilin biosynthesis, phytochromobilin formation, phytochromobilin synthesis Relationships: is a type of GO:0033014; is a type of dicarboxylic acid biosynthetic process [GO:0043650] Definition: The chemical reactions and pathways resulting in the formation of phytochromobilin, which involves the oxidative cleavage of heme by a heme oxygenase(HO) to form biliverdin IX alpha.